{
  "gene_name": "Tubulin gamma-2 chain",
  "term_label": "microtubule nucleator activity",
  "term_id": "GO:0140490",
  "gene": "UniProtKB:Q9NRH3",
  "gene_symbol": "TUBG2"
}